{
  "term_label": "DNA-binding transcription factor activity, RNA polymerase II-specific",
  "gene_name": "Zinc finger protein 257",
  "gene_symbol": "ZNF257",
  "term_id": "GO:0000981",
  "gene": "UniProtKB:Q9Y2Q1"
}